{
  "gene_name": "ERI1 exoribonuclease 3",
  "term_label": "cytosol",
  "gene_symbol": "ERI3",
  "term_id": "GO:0005829",
  "gene": "UniProtKB:O43414"
}